cortical microtubule organization [GO:0043622] (biological process) Definition: A process that is carried out at the cellular level which results in the assembly, arrangement of constituent parts, or disassembly of structures formed of microtubules and associated proteins in the cell cortex, i.e. just beneath the plasma membrane of a cell. Relationships: is_a GO:0030865; is a type of GO:0031122 Also known as: cortical microtubule cytoskeleton organization, cortical microtubule organisation, cortical microtubule organization and biogenesis Sources: GOC:curators, GOC:dph, GOC:jl, GOC:mah